{
  "gene": "UniProtKB:P98187",
  "term_id": "GO:0042376",
  "gene_symbol": "CYP4F8",
  "term_label": "phylloquinone catabolic process",
  "gene_name": "Cytochrome P450 4F8"
}